His-Purkinje system cell fate commitment [GO:0060934] (biological process) Definition: The commitment of cells to His-Purkinje cell fates and their capacity to differentiate into His-Purkinje cells. These cells form the fibers that regulate cardiac muscle contraction in the ventricles. Sources: GOC:mtg_heart Relationships: is_a cardiac cell fate commitment [GO:0060911]; is part of GO:0060932